high-density lipoprotein particle assembly [GO:0034380] (biological process) Definition: The non-covalent aggregation and arrangement of proteins and lipids to form a high-density lipoprotein particle. Also known as: HDL assembly Relationships: is a type of GO:0034377 Sources: GOC:BHF, GOC:mah Regulation: regulated by regulation of high-density lipoprotein particle assembly [GO:0090107]; RO_0002213 by positive regulation of high-density lipoprotein particle assembly [GO:0090108]